{
  "gene_symbol": "GSX2",
  "gene": "UniProtKB:Q9BZM3",
  "term_id": "UNKNOWN:0002",
  "term_label": "Unknown biological process",
  "gene_name": "GS homeobox 2"
}